{
  "term_label": "Arp2/3 complex-mediated actin nucleation",
  "gene_name": "Actin-related protein 2_3 complex subunit 3",
  "term_id": "GO:0034314",
  "gene": "UniProtKB:O15145",
  "gene_symbol": "ARPC3"
}